{
  "gene_name": "Protrudin",
  "gene": "UniProtKB:Q5T4F4",
  "gene_symbol": "ZFYVE27",
  "term_id": "GO:0048011",
  "term_label": "neurotrophin TRK receptor signaling pathway"
}